RNA metabolic process [GO:0016070] (biological process) Definition: The cellular chemical reactions and pathways involving RNA, ribonucleic acid, one of the two main type of nucleic acid, consisting of a long, unbranched macromolecule formed from ribonucleotides joined in 3',5'-phosphodiester linkage. Sources: ISBN:0198506732 Also known as: RNA metabolism Relationships: is a type of nucleic acid metabolic process [GO:0090304] Subtypes: GO:0000378, mitochondrial RNA metabolic process [GO:0000959], tRNA metabolic process [GO:0006399], RNA catabolic process [GO:0006401], RNA modification [GO:0009451], miRNA metabolic process [GO:0010586], mRNA metabolic process [GO:0016071], rRNA metabolic process [GO:0016072], snRNA metabolic process [GO:0016073], sno(s)RNA metabolic process [GO:0016074], GO:0032774, 21U-RNA metabolic process [GO:0034585], GO:0039703, RNA repair [GO:0042245], GO:0042868, RNA decapping [GO:0110154] Regulation: RO_0002211 by regulation of RNA metabolic process [GO:0051252]; negatively regulated by negative regulation of RNA metabolic process [GO:0051253]; positively regulated by positive regulation of RNA metabolic process [GO:0051254]